{
  "gene_symbol": "CTBP2",
  "gene_name": "C-terminal-binding protein 2",
  "term_id": "GO:0001221",
  "term_label": "transcription coregulator binding",
  "gene": "UniProtKB:P56545"
}